{
  "term_id": "GO:0071939",
  "gene_name": "Receptor for retinol uptake STRA6",
  "gene": "UniProtKB:Q9BX79",
  "term_label": "vitamin A import into cell",
  "gene_symbol": "STRA6"
}